{
  "gene_symbol": "MBTPS2",
  "term_label": "membrane protein intracellular domain proteolysis",
  "gene": "UniProtKB:O43462",
  "gene_name": "Membrane-bound transcription factor site-2 protease",
  "term_id": "GO:0031293"
}